cGMP biosynthetic process [GO:0006182] (biological process) Sources: ISBN:0198506732 Definition: The chemical reactions and pathways resulting in the formation of cyclic GMP, guanosine 3',5'-phosphate. Relationships: is a type of purine ribonucleotide biosynthetic process [GO:0009152]; is a type of cyclic nucleotide biosynthetic process [GO:0009190]; is a type of GO:0046068 Also known as: cGMP anabolism, cGMP biosynthesis, cGMP formation, cGMP synthesis